Golgi to endosome transport [GO:0006895] (biological process) Also known as: Golgi to endosome vesicle-mediated transport, TGN to endosome transport, trans-Golgi to endosome transport Relationships: is a type of GO:0006892; is_a cytosolic transport [GO:0016482] Definition: The directed movement of substances from the Golgi to early sorting endosomes. Clathrin vesicles transport substances from the trans-Golgi to endosomes. References: PMID:10873832 Sources: GOC:jl, ISBN:0716731363